fumarate reductase complex [GO:0045283] (cellular component) Relationships: is_a membrane protein complex [GO:0098796]; is a type of GO:0098803; is a type of catalytic complex [GO:1902494] Note: See also the molecular function term 'succinate dehydrogenase (ubiquinone) activity ; GO:0008177'. Definition: A membrane-bound flavoenzyme complex consisting of four subunits, A, B, C, and D. A and B comprise the membrane-extrinsic catalytic domain and C (InterPro:IPR003510; InterPro:IPR004224) and D (InterPro:IPR003418) link the catalytic centers to the electron-transport chain. This family consists of the 13 kDa hydrophobic subunit D. This component may be required to anchor the catalytic components of the fumarate reductase complex to the cytoplasmic membrane. Fumarate reductase couples the reduction of fumarate to succinate to the oxidation of quinol to quinone, in a reaction opposite to that catalyzed by the related complex II of the respiratory chain (succinate dehydrogenase-(ubiquinone)). Sources: InterPro:IPR003418, InterPro:IPR004224